sterol response element binding [GO:0032810] (molecular function) Also known as: SRE binding References: PMID:11994399 Sources: GOC:vk Definition: Binding to a sterol response element (SRE), a nonpalindromic sequence found in the promoters of genes involved in lipid metabolism. Relationships: is a type of GO:0000978